spine apparatus membrane [GO:0098897] (cellular component) Sources: GOC:mah Definition: The lipid bilayer surrounding the spine apparatus. Relationships: is a type of bounding membrane of organelle [GO:0098588]; is part of spine apparatus [GO:0097444]